oxidoreductase activity, acting on diphenols and related substances as donors, NAD or NADP as acceptor [GO:0016680] (MF) Subtypes: trans-acenaphthene-1,2-diol dehydrogenase activity [GO:0047062] Sources: GOC:jl Relationships: is a type of oxidoreductase activity, acting on diphenols and related substances as donors [GO:0016679] Definition: Catalysis of an oxidation-reduction (redox) reaction in which a diphenol, or related compound, acts as a hydrogen or electron donor and reduces NAD or NADP.